{
  "term_label": "phosphoglycerate mutase activity",
  "gene_symbol": "PGAM2",
  "term_id": "GO:0004619",
  "gene": "UniProtKB:P15259",
  "gene_name": "Phosphoglycerate mutase 2"
}